{
  "gene_name": "Hyaluronidase-2",
  "gene": "UniProtKB:Q12891",
  "term_label": "cytoplasmic vesicle",
  "term_id": "GO:0031410",
  "gene_symbol": "HYAL2"
}